{
  "gene_name": "Serotransferrin",
  "gene": "UniProtKB:P02787",
  "term_label": "Unknown molecular function",
  "gene_symbol": "TF",
  "term_id": "UNKNOWN:0001"
}